{
  "term_id": "GO:0004222",
  "gene": "UniProtKB:O75439",
  "gene_symbol": "PMPCB",
  "term_label": "metalloendopeptidase activity",
  "gene_name": "Mitochondrial-processing peptidase subunit beta"
}